{
  "term_id": "GO:0005737",
  "gene": "UniProtKB:O60443",
  "gene_symbol": "GSDME",
  "term_label": "cytoplasm",
  "gene_name": "Gasdermin-E"
}